{
  "term_id": "UNKNOWN:0001",
  "term_label": "Unknown molecular function",
  "gene_symbol": "ZNF385C",
  "gene": "UniProtKB:Q66K41",
  "gene_name": "Zinc finger protein 385C"
}